nuclear migration during mitotic telophase [GO:0090561] (biological process) References: PMID:23087209 Sources: GOC:vw Regulation: regulated by GO:1902852; RO_0002212 by negative regulation of nuclear migration during mitotic telophase [GO:1902853]; positively regulated by positive regulation of nuclear migration during mitotic telophase [GO:1902854] Relationships: is a type of GO:0030473 Definition: The dynein-driven microtubule based nuclear migration, whereby daughter nuclei are positioned away from the cell division site prior to cytokinesis.